regulation of neurotransmitter transport [GO:0051588] (biological process) Sources: GOC:ai Relationships: is a type of regulation of transport [GO:0051049]; regulates neurotransmitter transport [GO:0006836] Definition: Any process that modulates the frequency, rate or extent of the directed movement of a neurotransmitter into, out of or within a cell, or between cells, by means of some agent such as a transporter or pore. Subtypes: GO:0046928, regulation of neurotransmitter uptake [GO:0051580], negative regulation of neurotransmitter transport [GO:0051589], positive regulation of neurotransmitter transport [GO:0051590], GO:0099162